{
  "term_label": "GTPase activator activity",
  "gene": "UniProtKB:Q5VW22",
  "gene_name": "Arf-GAP with GTPase, ANK repeat and PH domain-containing protein 6",
  "gene_symbol": "AGAP6",
  "term_id": "GO:0005096"
}